{
  "term_label": "insulin-like growth factor receptor signaling pathway",
  "term_id": "GO:0048009",
  "gene": "UniProtKB:O75420",
  "gene_name": "GRB10-interacting GYF protein 1",
  "gene_symbol": "GIGYF1"
}